{
  "gene_name": "Pleckstrin",
  "term_id": "UNKNOWN:0001",
  "term_label": "Unknown molecular function",
  "gene_symbol": "PLEK",
  "gene": "UniProtKB:P08567"
}